polyamine transmembrane transporter activity [GO:0015203] (molecular function) Subtypes: spermine transmembrane transporter activity [GO:0000297], polyamine:proton antiporter activity [GO:0015312], ABC-type polyamine transporter activity [GO:0015417], GO:0015489, spermidine transmembrane transporter activity [GO:0015606] Relationships: is a type of GO:0022857; BFO_0000050 polyamine transmembrane transport [GO:1902047] Also known as: amine/amide/polyamine channel activity Definition: Enables the transfer of polyamines, organic compounds containing two or more amino groups, from one side of a membrane to the other. Sources: GOC:ai